{
  "term_label": "fatty acid metabolic process",
  "gene_symbol": "THEM4",
  "gene": "UniProtKB:Q5T1C6",
  "term_id": "GO:0006631",
  "gene_name": "Acyl-coenzyme A thioesterase THEM4"
}